{
  "term_label": "detection of chemical stimulus involved in sensory perception of smell",
  "gene_symbol": "OR2J3",
  "gene_name": "Olfactory receptor 2J3",
  "term_id": "GO:0050911",
  "gene": "UniProtKB:O76001"
}